transcription antitermination factor activity, RNA binding [GO:0001072] (molecular function) Relationships: is a type of transcription regulator activity [GO:0140110]; is part of GO:0031564 References: PMID:8332211 Sources: GOC:txnOH Also known as: RNA binding transcription antitermination factor activity Definition: Binds to RNA, typically within the nascent RNA transcript, to promote readthrough of a transcription termination site and thus extending the length of the RNA transcript produced. Examples of antitermination factors which bind the nascent RNA include the lambda N protein and the HIV-1 tat protein.